{
  "term_id": "GO:0050868",
  "gene_name": "Tyrosine-protein phosphatase non-receptor type 22",
  "gene_symbol": "PTPN22",
  "term_label": "negative regulation of T cell activation",
  "gene": "UniProtKB:Q9Y2R2"
}